regulation of linear element maturation [GO:0062123] (biological process) References: PMID:30640914 Relationships: is a type of regulation of chromosome organization [GO:0033044]; is a type of regulation of linear element assembly [GO:0090006]; regulates linear element maturation [GO:0062121] Definition: Any process that modulates the rate, frequency or extent of linear element maturation.